{
  "gene_symbol": "COL11A2",
  "gene": "UniProtKB:P13942",
  "term_id": "GO:0030199",
  "gene_name": "Collagen alpha-2(XI) chain",
  "term_label": "collagen fibril organization"
}